{
  "gene": "UniProtKB:P38405",
  "gene_symbol": "GNAL",
  "gene_name": "Guanine nucleotide-binding protein G(olf) subunit alpha",
  "term_label": "G protein-coupled receptor binding",
  "term_id": "GO:0001664"
}